{
  "gene_name": "Zinc finger transcription factor Trps1",
  "gene": "UniProtKB:Q9UHF7",
  "term_label": "RNA polymerase II transcription regulatory region sequence-specific DNA binding",
  "gene_symbol": "TRPS1",
  "term_id": "GO:0000977"
}